{
  "gene": "UniProtKB:A0A0J9YWU9",
  "gene_name": "Ig-like domain-containing protein (Fragment)",
  "term_id": "GO:0003823",
  "term_label": "antigen binding",
  "gene_symbol": "A0A0J9YWU9"
}